negative regulation of epiboly involved in gastrulation with mouth forming second [GO:1904087] (biological process) Also known as: down regulation of epiboly involved in gastrulation with mouth forming second, down-regulation of epiboly involved in gastrulation with mouth forming second, downregulation of epiboly involved in gastrulation with mouth forming second, inhibition of epiboly involved in gastrulation with mouth forming second References: PMID:24892953 Sources: GOC:TermGenie, GO_REF:0000058 Definition: Any process that stops, prevents or reduces the frequency, rate or extent of epiboly involved in gastrulation with mouth forming second. Relationships: is a type of GO:1904086; is a type of negative regulation of morphogenesis of an epithelium [GO:1905331]; negatively regulates epiboly involved in gastrulation with mouth forming second [GO:0055113]